{
  "term_id": "GO:0005615",
  "gene_symbol": "PRSS21",
  "term_label": "extracellular space",
  "gene": "UniProtKB:Q9Y6M0",
  "gene_name": "Testisin"
}